{
  "term_label": "negative regulation of transcription by RNA polymerase II",
  "gene": "UniProtKB:Q9BWX5",
  "term_id": "GO:0000122",
  "gene_symbol": "GATA5",
  "gene_name": "Transcription factor GATA-5"
}